{
  "gene": "UniProtKB:Q8TDY2",
  "gene_symbol": "RB1CC1",
  "term_id": "GO:1990316",
  "gene_name": "RB1-inducible coiled-coil protein 1",
  "term_label": "Atg1/ULK1 kinase complex"
}